{
  "gene_symbol": "UNK",
  "term_label": "cell morphogenesis involved in neuron differentiation",
  "gene": "UniProtKB:Q9C0B0",
  "gene_name": "RING finger protein unkempt homolog",
  "term_id": "GO:0048667"
}